{
  "term_label": "nucleoplasm",
  "gene_symbol": "HNRNPH3",
  "term_id": "GO:0005654",
  "gene_name": "Heterogeneous nuclear ribonucleoprotein H3",
  "gene": "UniProtKB:P31942"
}